{
  "gene_name": "Seven in absentia homolog 3",
  "gene_symbol": "SIAH3",
  "term_label": "ubiquitin conjugating enzyme binding",
  "term_id": "GO:0031624",
  "gene": "UniProtKB:Q8IW03"
}